desensitization of G protein-coupled receptor signaling pathway [GO:0002029] (biological process) Definition: The process that stops, prevents, or reduces the frequency, rate or extent of G protein-coupled receptor signaling pathway after prolonged stimulation with an agonist of the pathway. Relationships: is a type of negative adaptation of signaling pathway [GO:0022401]; is a type of negative regulation of G protein-coupled receptor signaling pathway [GO:0045744] References: PMID:8396717 Also known as: desensitisation of G-protein coupled receptor protein signalling pathway, desensitization of G-protein coupled receptor protein signaling pathway